2-methyl-6-geranylgeranyl-1,4-benzoquinol methyltransferase activity [GO:0102550] (molecular function) Relationships: is a type of methyltransferase activity [GO:0008168] Definition: Catalysis of the reaction: S-adenosyl-L-methionine + 2-methyl-6-geranylgeranyl-1,4-benzoquinol = S-adenosyl-L-homocysteine + 2,3-dimethyl-6-geranylgeranyl-1,4-benzoquinol + H+. Sources: EC:2.1.1.295, GOC:pz